{
  "term_label": "DNA-binding transcription factor activity, RNA polymerase II-specific",
  "gene": "UniProtKB:P78545",
  "gene_name": "ETS-related transcription factor Elf-3",
  "term_id": "GO:0000981",
  "gene_symbol": "ELF3"
}